{
  "gene_symbol": "GAREM1",
  "term_id": "UNKNOWN:0003",
  "gene_name": "GRB2-associated and regulator of MAPK protein 1",
  "term_label": "Unknown cellular component",
  "gene": "UniProtKB:Q9H706"
}